intramanchette transport [GO:1990953] (biological process) References: PMID:22319670, PMID:24440897, PMID:26792866 Sources: GOC:krc Relationships: is a type of GO:0031503; is_a protein transport along microtubule [GO:0098840]; is part of spermatid development [GO:0007286]; occurs in manchette [GO:0002177] Definition: The movement of vesicles and protein complexes carried out by molecular motors, kinesins and dynein, along the microtubule tracks within the manchette and by myosin along actin filaments. Also known as: IMT